{
  "term_label": "molecular adaptor activity",
  "gene_name": "Septin-12",
  "gene_symbol": "SEPTIN12",
  "term_id": "GO:0060090",
  "gene": "UniProtKB:Q8IYM1"
}